{
  "gene_name": "Platelet factor 4 variant",
  "gene": "UniProtKB:P10720",
  "term_id": "GO:0071222",
  "gene_symbol": "PF4V1",
  "term_label": "cellular response to lipopolysaccharide"
}